positive regulation of mitochondrial translational initiation [GO:0070134] (biological process) Definition: Any process that activates or increases the frequency, rate or extent of the process preceding formation of the peptide bond between the first two amino acids of a protein in a mitochondrion. Also known as: positive regulation of mitochondrial translation initiation Sources: GOC:mah Relationships: is a type of positive regulation of translational initiation [GO:0045948]; is a type of GO:0070131; is a type of regulation of mitochondrial translational initiation [GO:0070132]; RO_0002213 GO:0070124